{
  "term_label": "nucleus",
  "gene": "UniProtKB:Q7Z3H4",
  "gene_symbol": "SAMD7",
  "gene_name": "Sterile alpha motif domain-containing protein 7",
  "term_id": "GO:0005634"
}